large conductance calcium-activated potassium channel activity [GO:0060072] (molecular function) Regulation: negatively regulated by GO:1902607; positively regulated by positive regulation of large conductance calcium-activated potassium channel activity [GO:1902608] Relationships: is a type of calcium-activated potassium channel activity [GO:0015269] References: PMID:17115074 Sources: GOC:mtg_transport, ISBN:0815340729 Also known as: BK KCa channel activity, BK calcium-activated potassium channel activity, large conductance KCa channel activity, BK channel activity Definition: Enables the transmembrane transfer of potassium by a channel with a unit conductance of 100 to 220 picoSiemens that opens in response to stimulus by concerted actions of internal calcium ions and membrane potential. Large conductance calcium-activated potassium channels are less sensitive to calcium than are small or intermediate conductance calcium-activated potassium channels. Transport by a channel involves catalysis of facilitated diffusion of a solute (by an energy-independent process) involving passage through a transmembrane aqueous pore or channel, without evidence for a carrier-mediated mechanism.